{
  "term_id": "GO:0031624",
  "term_label": "ubiquitin conjugating enzyme binding",
  "gene": "UniProtKB:O60260",
  "gene_name": "E3 ubiquitin-protein ligase parkin",
  "gene_symbol": "PRKN"
}